{
  "gene_symbol": "COPZ1",
  "term_label": "retrograde vesicle-mediated transport, Golgi to endoplasmic reticulum",
  "term_id": "GO:0006890",
  "gene_name": "Coatomer subunit zeta-1",
  "gene": "UniProtKB:P61923"
}